{
  "gene": "UniProtKB:Q9BZZ5",
  "term_id": "GO:0043066",
  "gene_symbol": "API5",
  "term_label": "negative regulation of apoptotic process",
  "gene_name": "Apoptosis inhibitor 5"
}